{
  "gene": "UniProtKB:Q8IYD1",
  "gene_symbol": "GSPT2",
  "gene_name": "Eukaryotic peptide chain release factor GTP-binding subunit ERF3B",
  "term_id": "GO:0006412",
  "term_label": "translation"
}